{
  "term_id": "GO:0004984",
  "gene_symbol": "OR7G2",
  "gene_name": "Olfactory receptor 7G2",
  "gene": "UniProtKB:Q8NG99",
  "term_label": "olfactory receptor activity"
}